mitochondrial asparaginyl-tRNA aminoacylation [GO:0070145] (biological process) Sources: GOC:mah, GOC:mcc Definition: The process of coupling asparagine to asparaginyl-tRNA in a mitochondrion, catalyzed by asparaginyl-tRNA synthetase. In tRNA aminoacylation, the amino acid is first activated by linkage to AMP and then transferred to either the 2'- or the 3'-hydroxyl group of the 3'-adenosine residue of the tRNA. Relationships: is a type of asparaginyl-tRNA aminoacylation [GO:0006421]; is a type of GO:0070127